axonemal basal plate [GO:0097541] (cellular component) Relationships: is a type of cellular anatomical structure [GO:0110165]; is part of axoneme [GO:0005930] Definition: Part of the axoneme consisting of a highly electron-dense region at the distal end of the ciliary transition zone within the axonemal lumen at which the axonemal central pair of microtubules is connected to the rest of the axonemal structure. References: PMID:23352055, PMID:4554367 Sources: GOC:cilia Also known as: basal plate, axoneme basal plate